nucleus ambiguus development [GO:0021745] (biological process) Definition: The process whose specific outcome is the progression of the nucleus ambiguus over time, from its formation to the mature structure. Relationships: is a type of neural nucleus development [GO:0048857]; is part of medulla oblongata development [GO:0021550] Sources: GOC:cls, GOC:curators, GOC:dgh, GOC:dph, GOC:jid